{
  "gene_name": "Huntingtin-associated protein 1",
  "term_label": "mitochondrion distribution",
  "term_id": "GO:0048311",
  "gene_symbol": "HAP1",
  "gene": "UniProtKB:P54257"
}